{
  "term_id": "UNKNOWN:0002",
  "gene_symbol": "CCDC175",
  "term_label": "Unknown biological process",
  "gene_name": "Coiled-coil domain-containing protein 175",
  "gene": "UniProtKB:P0C221"
}